{
  "gene_symbol": "PPIA",
  "term_id": "GO:0016018",
  "gene": "UniProtKB:P62937",
  "term_label": "cyclosporin A binding",
  "gene_name": "Peptidyl-prolyl cis-trans isomerase A"
}